{
  "gene": "UniProtKB:Q8NFQ5",
  "term_id": "UNKNOWN:0001",
  "gene_name": "BPI fold-containing family B member 6",
  "term_label": "Unknown molecular function",
  "gene_symbol": "BPIFB6"
}